{
  "term_id": "GO:0006367",
  "term_label": "transcription initiation at RNA polymerase II promoter",
  "gene": "UniProtKB:Q6P1X5",
  "gene_symbol": "TAF2",
  "gene_name": "Transcription initiation factor TFIID subunit 2"
}